{
  "term_label": "protein localization to chromosome, telomeric region",
  "term_id": "GO:0070198",
  "gene_name": "Telomeric repeat-binding factor 2",
  "gene": "UniProtKB:Q15554",
  "gene_symbol": "TERF2"
}